peptidase complex [GO:1905368] (cellular component) References: PMID:1689240 Sources: GOC:TermGenie, GOC:bhm, GO_REF:0000088 Note: An example of this is PLAU in human (UniProt symbol P00749) in PMID:1689240 (inferred from direct assay). Definition: A protein complex which is capable of peptidase activity. Relationships: is a type of catalytic complex [GO:1902494] Also known as: protease complex, tryptase complex Subtypes: GO:0000124, m-AAA complex [GO:0005745], glutathione hydrolase complex [GO:0061672], PNGase complex [GO:0120125], serine-type peptidase complex [GO:1905286], endopeptidase complex [GO:1905369], GO:1990850, GO:1990861